{
  "gene_name": "Centromere protein O",
  "term_id": "GO:0031511",
  "gene_symbol": "CENPO",
  "gene": "UniProtKB:Q9BU64",
  "term_label": "Mis6-Sim4 complex"
}